hemolysis in another organism [GO:0044179] (biological process) Also known as: hemolysis in other organism, hemolysis of RBCs in other organism, hemolysis of cells in other organism, hemolysis of erythrocytes in other organism, hemolysis of red blood cells in other organism, envenomation resulting in hemolysis in another organism, envenomation resulting in hemolysis in other organism References: PMID:21590705 Sources: GOC:jl Definition: The cytolytic destruction of red blood cells, with the release of intracellular hemoglobin, in one organism by another. Relationships: is a type of cytolysis in another organism [GO:0051715]